{
  "gene_name": "Immunoglobulin lambda variable 4-69",
  "term_id": "UNKNOWN:0001",
  "term_label": "Unknown molecular function",
  "gene_symbol": "IGLV4-69",
  "gene": "UniProtKB:A0A075B6H9"
}